{
  "gene_symbol": "CISD1",
  "term_id": "GO:0051537",
  "gene_name": "CDGSH iron-sulfur domain-containing protein 1",
  "gene": "UniProtKB:Q9NZ45",
  "term_label": "2 iron, 2 sulfur cluster binding"
}